luteolin 7-O-glucuronosyltransferase activity [GO:0050064] (molecular function) Also known as: luteolin 7-O-glucoronosyltransferase activity, LGT, UDP-glucuronate:luteolin 7-O-glucuronosyltransferase activity, UDPglucuronate:luteolin 7-O-glucuronosyltransferase activity, uridine diphosphoglucuronate-luteolin 7-O-glucuronosyltransferase activity Definition: Catalysis of the reaction: luteolin + UDP-alpha-D-glucuronate = luteolin 7-O-beta-D-glucosiduronate + UDP. Sources: EC:2.4.1.189, RHEA:10568 Relationships: is a type of glucuronosyltransferase activity [GO:0015020]